{
  "gene": "UniProtKB:P51688",
  "term_label": "N-sulfoglucosamine sulfohydrolase activity",
  "gene_name": "N-sulphoglucosamine sulphohydrolase",
  "term_id": "GO:0016250",
  "gene_symbol": "SGSH"
}